cellular response to mannose [GO:1905583] (biological process) References: PMID:16699509 Sources: GOC:TermGenie, GO_REF:0000071 Definition: Any process that results in a change in state or activity of a cell (in terms of movement, secretion, enzyme production, gene expression, etc.) as a result of a mannose stimulus. Relationships: is a type of GO:0071331; is a type of GO:1905582